positive regulation of T cell anergy [GO:0002669] (biological process) Definition: Any process that activates or increases the frequency, rate, or extent of T cell anergy. Sources: GOC:add Also known as: positive regulation of T lymphocyte anergy, positive regulation of T-cell anergy, positive regulation of T-lymphocyte anergy, up regulation of T cell anergy, up-regulation of T cell anergy, upregulation of T cell anergy, activation of T cell anergy, stimulation of T cell anergy Relationships: is a type of positive regulation of T cell tolerance induction [GO:0002666]; is a type of regulation of T cell anergy [GO:0002667]; is a type of positive regulation of lymphocyte anergy [GO:0002913]; positively regulates T cell anergy [GO:0002870]